{
  "term_id": "GO:0005829",
  "term_label": "cytosol",
  "gene": "UniProtKB:Q07352",
  "gene_name": "mRNA decay activator protein ZFP36L1",
  "gene_symbol": "ZFP36L1"
}